{
  "gene_symbol": "TSEN34",
  "gene": "UniProtKB:Q9BSV6",
  "term_label": "tRNA-intron lyase activity",
  "term_id": "GO:0000213",
  "gene_name": "tRNA-splicing endonuclease subunit Sen34"
}